{
  "gene_symbol": "C12orf76",
  "gene": "UniProtKB:Q8N812",
  "term_label": "Unknown cellular component",
  "term_id": "UNKNOWN:0003",
  "gene_name": "Uncharacterized protein C12orf76"
}